{
  "gene_name": "Fibrinogen-like protein 1",
  "gene": "UniProtKB:Q08830",
  "term_id": "GO:0050776",
  "gene_symbol": "FGL1",
  "term_label": "regulation of immune response"
}